positive regulation of epidermal growth factor receptor signaling pathway [GO:0045742] (biological process) Relationships: is a type of regulation of epidermal growth factor receptor signaling pathway [GO:0042058]; is a type of positive regulation of ERBB signaling pathway [GO:1901186]; positively regulates epidermal growth factor receptor signaling pathway [GO:0007173] Sources: GOC:go_curators Definition: Any process that activates or increases the frequency, rate or extent of epidermal growth factor receptor signaling pathway activity. Also known as: positive regulation of EGF receptor signaling pathway, positive regulation of EGF receptor signalling pathway, positive regulation of EGFR signaling pathway, up regulation of epidermal growth factor receptor signaling pathway, up-regulation of epidermal growth factor receptor signaling pathway, upregulation of epidermal growth factor receptor signaling pathway, activation of epidermal growth factor receptor signaling pathway, stimulation of epidermal growth factor receptor signaling pathway Subtypes: positive regulation of epidermal growth factor receptor signaling pathway involved in heart process [GO:1905284]